regulation of galactotriose transport [GO:1900291] (biological process) Relationships: is a type of regulation of transport [GO:0051049]; regulates galactotriose transport [GO:2001093] Subtypes: negative regulation of galactotriose transport [GO:1900292], positive regulation of galactotriose transport [GO:1900293] Sources: GOC:TermGenie, GOC:mengo_curators Definition: Any process that modulates the frequency, rate or extent of galactotriose transport.